{
  "gene": "UniProtKB:Q96LD1",
  "term_label": "Unknown molecular function",
  "gene_symbol": "SGCZ",
  "term_id": "UNKNOWN:0001",
  "gene_name": "Zeta-sarcoglycan"
}